interleukin-16 binding [GO:0042011] (molecular function) Relationships: is a type of cytokine binding [GO:0019955] Sources: GOC:jl Definition: Binding to interleukin-16. Also known as: IL-16 binding